regulation of synaptic transmission, glutamatergic [GO:0051966] (biological process) Subtypes: negative regulation of synaptic transmission, glutamatergic [GO:0051967], positive regulation of synaptic transmission, glutamatergic [GO:0051968], GO:1903294 Definition: Any process that modulates the frequency, rate or extent of glutamatergic synaptic transmission, the process of communication from a neuron to another neuron across a synapse using the neurotransmitter glutamate. Sources: GOC:ai Relationships: is a type of modulation of chemical synaptic transmission [GO:0050804]; regulates synaptic transmission, glutamatergic [GO:0035249]